myeloid cell apoptotic process [GO:0033028] (biological process) Definition: Any apoptotic process in a myeloid cell, a cell of the monocyte, granulocyte, mast cell, megakaryocyte, or erythroid lineage. References: PMID:11292031, PMID:15330259, PMID:17133093 Sources: CL:0000763, GOC:add, GOC:mtg_apoptosis Also known as: apoptosis of myeloid cells, myeloid cell apoptosis Relationships: is a type of apoptotic process [GO:0006915] Subtypes: GO:0001781, mast cell apoptotic process [GO:0033024], macrophage apoptotic process [GO:0071888], erythrocyte apoptotic process [GO:1902217] Regulation: regulated by regulation of myeloid cell apoptotic process [GO:0033032]; negatively regulated by GO:0033033; RO_0002213 by GO:0033034